{
  "gene": "UniProtKB:O60879",
  "term_id": "GO:0005884",
  "gene_symbol": "DIAPH2",
  "term_label": "actin filament",
  "gene_name": "Protein diaphanous homolog 2"
}